{
  "gene_symbol": "DEFB108B",
  "term_id": "UNKNOWN:0001",
  "term_label": "Unknown molecular function",
  "gene": "UniProtKB:Q8NET1",
  "gene_name": "Beta-defensin 108B"
}